{
  "gene_name": "Suppressor of fused homolog",
  "gene": "UniProtKB:Q9UMX1",
  "gene_symbol": "SUFU",
  "term_id": "GO:0045879",
  "term_label": "negative regulation of smoothened signaling pathway"
}